cholesterol efflux [GO:0033344] (biological process) Regulation: regulated by GO:0010874; positively regulated by positive regulation of cholesterol efflux [GO:0010875]; negatively regulated by negative regulation of cholesterol efflux [GO:0090370] Also known as: cholesterol export Relationships: is a type of cholesterol transport [GO:0030301] Definition: The directed movement of cholesterol, cholest-5-en-3-beta-ol, out of a cell or organelle. Sources: GOC:sart